myo-inositol transmembrane transporter activity [GO:0005365] (MF) Subtypes: myo-inositol:proton symporter activity [GO:0005366], myo-inositol:sodium symporter activity [GO:0005367] Also known as: vitamin Bh transporter activity Sources: GOC:ai Relationships: is a type of polyol transmembrane transporter activity [GO:0015166]; is part of myo-inositol transport [GO:0015798] Definition: Enables the transfer of myo-inositol from one side of a membrane to the other. Myo-inositol is 1,2,3,4,5/4,6-cyclohexanehexol, a growth factor for animals and microorganisms.